{
  "term_id": "GO:0042254",
  "gene": "UniProtKB:O15381",
  "gene_name": "Nuclear valosin-containing protein-like",
  "term_label": "ribosome biogenesis",
  "gene_symbol": "NVL"
}